positive regulation of gonad development [GO:1905941] (biological process) Definition: Any process that activates or increases the frequency, rate or extent of gonad development. References: PMID:15342467 Sources: GOC:TermGenie, GO_REF:0000058 Also known as: positive regulation of gonadogenesis, up regulation of gonad development, up regulation of gonadogenesis, up-regulation of gonad development, up-regulation of gonadogenesis, upregulation of gonad development, upregulation of gonadogenesis, activation of gonad development, activation of gonadogenesis Relationships: is_a positive regulation of developmental process [GO:0051094]; is a type of positive regulation of multicellular organismal process [GO:0051240]; is a type of GO:1905939; is a type of positive regulation of reproductive process [GO:2000243]; positively regulates gonad development [GO:0008406] Subtypes: positive regulation of male gonad development [GO:2000020], positive regulation of female gonad development [GO:2000196]